cellular response to very-low-density lipoprotein particle stimulus [GO:0090731] (biological process) Relationships: is a type of response to lipoprotein particle [GO:0055094]; is a type of cellular response to lipoprotein particle stimulus [GO:0071402] Regulation: negatively regulated by negative regulation of cellular response to very-low-density lipoprotein particle stimulus [GO:1905888]; positively regulated by positive regulation of cellular response to very-low-density lipoprotein particle stimulus [GO:1905889]; regulated by regulation of cellular response to very-low-density lipoprotein particle stimulus [GO:1905890] Also known as: cellular response to VLDL particle stimulus Sources: GOC:aruk, GOC:bc Definition: Any process that results in a change in state or activity of a cell (in terms of movement, secretion, enzyme production, gene expression, etc.) as a result of a very-low-density lipoprotein particle stimulus.